{
  "gene_symbol": "FRAS1",
  "gene": "UniProtKB:Q86XX4",
  "gene_name": "Extracellular matrix organizing protein FRAS1",
  "term_id": "UNKNOWN:0001",
  "term_label": "Unknown molecular function"
}